cyclic photosynthetic phosphorylation [GO:0009778] (biological process) Definition: A photosynthetic phosphorylation process in which ATP synthesis is driven by a proton gradient generated across the thylakoid membrane. Involves only photosystem I. Relationships: is a type of photosynthetic phosphorylation [GO:0009777] Sources: ISBN:0198547684